{
  "term_id": "UNKNOWN:0003",
  "gene_symbol": "GPT2",
  "gene": "UniProtKB:Q8TD30",
  "term_label": "Unknown cellular component",
  "gene_name": "Alanine aminotransferase 2"
}